positive regulation of copper ion transmembrane transport [GO:1902313] (biological process) Also known as: positive regulation of copper cation transmembrane transport, positive regulation of copper ion membrane transport, up regulation of copper cation transmembrane transport, up regulation of copper ion membrane transport, up regulation of copper ion transmembrane transport, up-regulation of copper cation transmembrane transport, up-regulation of copper ion membrane transport, up-regulation of copper ion transmembrane transport, upregulation of copper cation transmembrane transport, upregulation of copper ion membrane transport, upregulation of copper ion transmembrane transport, activation of copper cation transmembrane transport, activation of copper ion membrane transport, activation of copper ion transmembrane transport References: PMID:21489137 Sources: GOC:TermGenie, GOC:di Relationships: is a type of regulation of copper ion transmembrane transport [GO:1902311]; is a type of positive regulation of cation transmembrane transport [GO:1904064]; positively regulates copper ion transmembrane transport [GO:0035434] Definition: Any process that activates or increases the frequency, rate or extent of copper ion transmembrane transport.